regulation of N-terminal peptidyl-methionine acetylation [GO:1904663] (biological process) Subtypes: GO:1904664, positive regulation of N-terminal peptidyl-methionine acetylation [GO:1904665] Relationships: is a type of GO:1901983; is a type of regulation of protein maturation [GO:1903317]; regulates N-terminal peptidyl-methionine acetylation [GO:0017196] References: PMID:20807799 Sources: GOC:TermGenie, GO_REF:0000058 Definition: Any process that modulates the frequency, rate or extent of N-terminal peptidyl-methionine acetylation.